{
  "gene": "UniProtKB:Q8NC26",
  "term_id": "GO:0000978",
  "gene_name": "Zinc finger protein 114",
  "term_label": "RNA polymerase II cis-regulatory region sequence-specific DNA binding",
  "gene_symbol": "ZNF114"
}